{
  "term_label": "Unknown cellular component",
  "gene_name": "Cysteine-rich protein 2",
  "gene_symbol": "CRIP2",
  "term_id": "UNKNOWN:0003",
  "gene": "UniProtKB:P52943"
}